E-box binding [GO:0070888] (molecular function) Also known as: E-box promoter binding References: PMID:11812799 Sources: GOC:BHF, GOC:vk Definition: Binding to an E-box, a DNA motif with the consensus sequence CANNTG that is found in the promoters of a wide array of genes expressed in neurons, muscle and other tissues. Relationships: is a type of RNA polymerase II cis-regulatory region sequence-specific DNA binding [GO:0000978]